{
  "gene_symbol": "PIK3C3",
  "term_id": "GO:0016020",
  "gene_name": "Phosphatidylinositol 3-kinase catalytic subunit type 3",
  "gene": "UniProtKB:Q8NEB9",
  "term_label": "membrane"
}